{
  "gene": "UniProtKB:Q8N3J5",
  "term_label": "protein serine/threonine phosphatase activity",
  "gene_symbol": "PPM1K",
  "gene_name": "Protein phosphatase 1K, mitochondrial",
  "term_id": "GO:0004722"
}